{
  "gene_name": "Casein kinase I isoform gamma-2",
  "gene": "UniProtKB:P78368",
  "gene_symbol": "CSNK1G2",
  "term_label": "plasma membrane",
  "term_id": "GO:0005886"
}